{
  "gene_name": "Protein THEMIS2",
  "gene_symbol": "THEMIS2",
  "term_label": "nucleus",
  "term_id": "GO:0005634",
  "gene": "UniProtKB:Q5TEJ8"
}